post-anaphase microtubule array organization [GO:1904186] (biological process) Relationships: is a type of cellular component organization [GO:0016043] Also known as: PAA organization, post-anaphase array organization, post-anaphase microtubule array organisation References: PMID:15004232 Sources: GOC:TermGenie Definition: A process that is carried out at the cellular level which results in the assembly, arrangement of constituent parts, or disassembly ofa post-anaphase microtubule array.